{
  "term_id": "GO:0034497",
  "gene": "UniProtKB:Q5MNZ9",
  "gene_name": "WD repeat domain phosphoinositide-interacting protein 1",
  "term_label": "protein localization to phagophore assembly site",
  "gene_symbol": "WIPI1"
}